{
  "term_label": "ubiquitin conjugating enzyme activity",
  "gene_symbol": "UBE2N",
  "gene": "UniProtKB:P61088",
  "term_id": "GO:0061631",
  "gene_name": "Ubiquitin-conjugating enzyme E2 N"
}